cellotriose metabolic process [GO:2000893] (biological process) Subtypes: cellotriose catabolic process [GO:2000894] Also known as: cellotriose metabolism Sources: GOC:mengo_curators Definition: The chemical reactions and pathways involving a cellotriose. Relationships: is a type of oligosaccharide metabolic process [GO:0009311]